negative regulation of hormone biosynthetic process [GO:0032353] (biological process) Sources: GOC:ai Definition: Any process that stops, prevents, or reduces the frequency, rate or extent of the chemical reactions and pathways resulting in the formation of hormones. Relationships: is a type of negative regulation of biosynthetic process [GO:0009890]; is a type of negative regulation of hormone metabolic process [GO:0032351]; is a type of regulation of hormone biosynthetic process [GO:0046885]; negatively regulates hormone biosynthetic process [GO:0042446] Subtypes: GO:0045968, negative regulation of steroid hormone biosynthetic process [GO:0090032], negative regulation of indoleacetic acid biosynthetic process via tryptophan [GO:1901997], negative regulation of estrogen biosynthetic process [GO:1904077], negative regulation of androgen biosynthetic process [GO:2000180], negative regulation of progesterone biosynthetic process [GO:2000183] Also known as: down regulation of hormone biosynthetic process, down-regulation of hormone biosynthetic process, downregulation of hormone biosynthetic process, inhibition of hormone biosynthetic process